actin tubule [GO:0031003] (cellular component) Definition: A cellular structure, approximately 13 nm in diameter, consisting of three actin filaments bundled together. Relationships: is_a GO:0032432; is part of GO:0031002 Sources: GOC:kp